{
  "gene_name": "Histone-lysine N-methyltransferase EZH2",
  "term_id": "GO:0035098",
  "term_label": "ESC/E(Z) complex",
  "gene": "UniProtKB:Q15910",
  "gene_symbol": "EZH2"
}